{
  "gene_symbol": "MAPRE2",
  "term_label": "spindle assembly",
  "gene_name": "Microtubule-associated protein RP_EB family member 2",
  "gene": "UniProtKB:Q15555",
  "term_id": "GO:0051225"
}